host peribacteroid fluid [GO:0043665] (cellular component) Relationships: is a type of host cell part [GO:0033643]; is part of GO:0043663 Sources: GOC:cc Definition: The soluble material inside the peribacteroid membrane, but outside of the bacteroid, within a bacteroid-containing symbiosome of a host cell.